teichoic acid transport [GO:0015777] (biological process) Sources: GOC:ai Relationships: is a type of carbohydrate derivative transport [GO:1901264] Definition: The directed movement of teichoic acid into, out of or within a cell, or between cells, by means of some agent such as a transporter or pore. Teichoic acid is any polymer occurring in the cell wall, membrane or capsule of Gram-positive bacteria and containing chains of glycerol phosphate or ribitol phosphate residues.